{
  "gene": "UniProtKB:P31321",
  "gene_name": "cAMP-dependent protein kinase type I-beta regulatory subunit",
  "term_id": "GO:0007189",
  "gene_symbol": "PRKAR1B",
  "term_label": "adenylate cyclase-activating G protein-coupled receptor signaling pathway"
}